{
  "gene_symbol": "SOX17",
  "term_label": "vasculogenesis",
  "gene_name": "Transcription factor SOX-17",
  "term_id": "GO:0001570",
  "gene": "UniProtKB:Q9H6I2"
}